xenobiotic transport across blood-brain barrier [GO:1990962] (biological process) References: PMID:25053619 Relationships: is a type of xenobiotic transport [GO:0042908]; is a type of transport across blood-brain barrier [GO:0150104] Also known as: drug transport across blood-brain barrier Definition: The directed movement of a xenobiotic through the blood-brain barrier.